{
  "gene_name": "Homeobox even-skipped homolog protein 1",
  "gene": "UniProtKB:P49640",
  "gene_symbol": "EVX1",
  "term_label": "RNA polymerase II cis-regulatory region sequence-specific DNA binding",
  "term_id": "GO:0000978"
}